{
  "term_label": "positive regulation of filopodium assembly",
  "gene": "UniProtKB:Q8NEV4",
  "term_id": "GO:0051491",
  "gene_name": "Myosin-IIIa",
  "gene_symbol": "MYO3A"
}